intracellular organelle [GO:0043229] (cellular component) Sources: GOC:go_curators Definition: Organized structure of distinctive morphology and function, occurring within the cell. Includes the nucleus, mitochondria, plastids, vacuoles, vesicles, ribosomes and the cytoskeleton. Excludes the plasma membrane. Subtypes: intracellular membrane-bounded organelle [GO:0043231], intracellular membraneless organelle [GO:0043232] Relationships: is a type of organelle [GO:0043226]; BFO_0000050 intracellular anatomical structure [GO:0005622]